{
  "gene": "UniProtKB:Q9HAN9",
  "term_id": "GO:0000309",
  "term_label": "nicotinamide-nucleotide adenylyltransferase activity",
  "gene_symbol": "NMNAT1",
  "gene_name": "Nicotinamide_nicotinic acid mononucleotide adenylyltransferase 1"
}